{
  "gene_name": "EF-hand domain-containing protein D2",
  "gene_symbol": "EFHD2",
  "gene": "UniProtKB:Q96C19",
  "term_label": "Unknown cellular component",
  "term_id": "UNKNOWN:0003"
}